{
  "gene": "UniProtKB:Q5T280",
  "gene_name": "Putative methyltransferase C9orf114",
  "gene_symbol": "SPOUT1",
  "term_id": "GO:0035196",
  "term_label": "miRNA processing"
}